lipopolysaccharide-mediated virion attachment to host cell [GO:0039638] (BP) References: PMID:12837775 Sources: GOC:bf, GOC:bm Definition: The process by which a virion attaches to a host cell by binding to a lipopolysaccharide (LPS) on the host cell surface. Relationships: is a type of virion attachment to host cell [GO:0019062]; has part lipopolysaccharide binding [GO:0001530] Also known as: LPS binding involved in viral attachment to host cell, lipopolysaccharide binding involved in viral attachment to host cell, virion attachment, binding to host lipopolysaccharide